{
  "term_label": "calcium ion binding",
  "gene_symbol": "PLA2G2E",
  "gene": "UniProtKB:Q9NZK7",
  "term_id": "GO:0005509",
  "gene_name": "Group IIE secretory phospholipase A2"
}